negative regulation of neutrophil mediated killing of symbiont cell [GO:0070955] (BP) Subtypes: negative regulation of neutrophil mediated killing of bacterium [GO:0070956], negative regulation of neutrophil mediated killing of fungus [GO:0070959] Definition: Any process that decreases the frequency, rate or extent of the directed killing of a symbiont target cell by a neutrophil. Relationships: is a type of GO:0002832; is a type of GO:0031348; is a type of GO:0032102; is a type of negative regulation of killing of cells of another organism [GO:0051711]; is a type of GO:0070949; is a type of negative regulation of neutrophil mediated cytotoxicity [GO:0070954]; negatively regulates neutrophil-mediated killing of symbiont cell [GO:0070943] Also known as: down regulation of neutrophil mediated killing of symbiont cell, down-regulation of neutrophil mediated killing of symbiont cell, downregulation of neutrophil mediated killing of symbiont cell, inhibition of neutrophil mediated killing of symbiont cell Sources: GOC:add, GOC:mah